{
  "gene": "UniProtKB:P19022",
  "term_label": "synapse assembly",
  "gene_name": "Cadherin-2",
  "term_id": "GO:0007416",
  "gene_symbol": "CDH2"
}